{
  "gene_symbol": "S100A14",
  "gene": "UniProtKB:Q9HCY8",
  "term_id": "GO:0034142",
  "term_label": "toll-like receptor 4 signaling pathway",
  "gene_name": "Protein S100-A14"
}